protein delipidation [GO:0051697] (biological process) Definition: The breakage of covalent bonds to detach lipid groups from a protein. Sources: GOC:ai Relationships: is a type of GO:0036211